D-lysine transaminase activity [GO:0043911] (molecular function) Definition: Catalysis of the reaction: D-lysine + 2-oxoglutarate = L-glutamate + 6-amino-2-oxohexanoate. Relationships: is a type of transaminase activity [GO:0008483] References: PMID:17259313 Sources: GOC:jl Also known as: D-lysine aminotransferase activity